{
  "gene_symbol": "DTWD2",
  "gene": "UniProtKB:Q8NBA8",
  "gene_name": "tRNA-uridine aminocarboxypropyltransferase 2",
  "term_id": "UNKNOWN:0002",
  "term_label": "Unknown biological process"
}